{
  "gene_symbol": "CHST11",
  "gene_name": "Carbohydrate sulfotransferase 11",
  "gene": "UniProtKB:Q9NPF2",
  "term_label": "Unknown cellular component",
  "term_id": "UNKNOWN:0003"
}